{
  "term_label": "cytoplasm",
  "term_id": "GO:0005737",
  "gene_symbol": "LOC107987545",
  "gene_name": "DH domain-containing protein",
  "gene": "UniProtKB:A0A2R8YFR7"
}